{
  "gene": "UniProtKB:Q9Y2L5",
  "gene_name": "Trafficking protein particle complex subunit 8",
  "gene_symbol": "TRAPPC8",
  "term_label": "TRAPPIII protein complex",
  "term_id": "GO:1990072"
}